{
  "term_id": "GO:0034237",
  "gene_symbol": "TDRD10",
  "gene_name": "Tudor domain-containing protein 10",
  "gene": "UniProtKB:Q5VZ19",
  "term_label": "protein kinase A regulatory subunit binding"
}